{
  "gene_symbol": "CD300LG",
  "gene_name": "CMRF35-like molecule 9",
  "term_label": "plasma membrane",
  "gene": "UniProtKB:Q6UXG3",
  "term_id": "GO:0005886"
}